{
  "gene_name": "NudC domain-containing protein 3",
  "gene": "UniProtKB:Q8IVD9",
  "gene_symbol": "NUDCD3",
  "term_label": "protein folding",
  "term_id": "GO:0006457"
}